{
  "gene": "UniProtKB:Q5T447",
  "term_id": "GO:0004842",
  "gene_symbol": "HECTD3",
  "gene_name": "E3 ubiquitin-protein ligase HECTD3",
  "term_label": "ubiquitin-protein transferase activity"
}